{
  "term_id": "GO:0030215",
  "gene_symbol": "SEMA4A",
  "term_label": "semaphorin receptor binding",
  "gene_name": "Semaphorin-4A",
  "gene": "UniProtKB:Q9H3S1"
}